myelin maintenance [GO:0043217] (biological process) Definition: The process of preserving the structure and function of mature myelin. This includes maintaining the compact structure of myelin necessary for its electrical insulating characteristics as well as the structure of non-compact regions such as Schmidt-Lantermann clefts and paranodal loops. This does not include processes responsible for maintaining the nodes of Ranvier, which are not part of the myelin sheath. Sources: GOC:dgh Relationships: is a type of plasma membrane organization [GO:0007009]; BFO_0000050 myelination [GO:0042552] Subtypes: central nervous system myelin maintenance [GO:0032286], peripheral nervous system myelin maintenance [GO:0032287] Also known as: myelin sheath maintenance